reproductive structure development [GO:0048608] (BP) Sources: GOC:dph, GOC:isa_complete, GOC:jid Subtypes: gonad development [GO:0008406], fruit development [GO:0010154], GO:0030850, plant-type ovary development [GO:0035670], GO:0048316, genitalia development [GO:0048806], uterus development [GO:0060065], oviduct development [GO:0060066], cervix development [GO:0060067], seminal vesicle development [GO:0061107], seminiferous tubule development [GO:0072520], GO:0075259, GO:0090567, fungal sorus development [GO:0099121], baculum development [GO:1990375] Definition: The reproductive developmental process whose specific outcome is the progression of somatic structures that will be used in the process of creating new individuals from one or more parents, from their formation to the mature structures. Relationships: is a type of developmental process involved in reproduction [GO:0003006]; is a type of anatomical structure development [GO:0048856]; is part of reproductive system development [GO:0061458]